{
  "gene": "UniProtKB:A0A286YFK9",
  "gene_name": "Small integral membrane protein 38",
  "gene_symbol": "SMIM38",
  "term_label": "Unknown molecular function",
  "term_id": "UNKNOWN:0001"
}